{
  "term_id": "GO:0005667",
  "term_label": "transcription regulator complex",
  "gene_name": "Transducin-like enhancer protein 1",
  "gene_symbol": "TLE1",
  "gene": "UniProtKB:Q04724"
}